{
  "gene": "UniProtKB:O14641",
  "term_label": "frizzled binding",
  "term_id": "GO:0005109",
  "gene_name": "Segment polarity protein dishevelled homolog DVL-2",
  "gene_symbol": "DVL2"
}